{
  "term_id": "GO:0035259",
  "gene_name": "Nuclear receptor subfamily 4 group A member 1",
  "term_label": "nuclear glucocorticoid receptor binding",
  "gene": "UniProtKB:P22736",
  "gene_symbol": "NR4A1"
}